{
  "gene_symbol": "PLEKHG3",
  "term_label": "guanyl-nucleotide exchange factor activity",
  "gene": "UniProtKB:A1L390",
  "gene_name": "Pleckstrin homology domain-containing family G member 3",
  "term_id": "GO:0005085"
}